monoatomic anion transmembrane transport [GO:0098656] (biological process) Definition: The process in which a monoatomic anion is transported across a membrane. Monatomic anions (also called simple anions) are negatively charged ions consisting of exactly one atom. Sources: GOC:dos, GOC:vw Subtypes: GO:1902476, fluoride transmembrane transport [GO:1903424], iodide transmembrane transport [GO:1904200] Also known as: anion transmembrane transport, ATP hydrolysis coupled anion transmembrane transport Relationships: is a type of GO:0006820; is a type of monoatomic ion transmembrane transport [GO:0034220] Regulation: regulated by regulation of monoatomic anion transmembrane transport [GO:1903959]; negatively regulated by negative regulation of anion transmembrane transport [GO:1903960]; positively regulated by GO:1903961